{
  "gene_name": "Protein SCO2 homolog, mitochondrial",
  "term_id": "UNKNOWN:0003",
  "gene_symbol": "SCO2",
  "term_label": "Unknown cellular component",
  "gene": "UniProtKB:O43819"
}